{
  "term_id": "GO:0005737",
  "gene": "UniProtKB:Q13509",
  "term_label": "cytoplasm",
  "gene_name": "Tubulin beta-3 chain",
  "gene_symbol": "TUBB3"
}